{
  "term_id": "GO:0031647",
  "gene_name": "Ubiquitin carboxyl-terminal hydrolase 1",
  "gene_symbol": "USP1",
  "gene": "UniProtKB:O94782",
  "term_label": "regulation of protein stability"
}